{
  "gene_name": "Deoxycytidylate deaminase",
  "term_id": "GO:0005737",
  "gene_symbol": "DCTD",
  "term_label": "cytoplasm",
  "gene": "UniProtKB:P32321"
}